{
  "term_id": "UNKNOWN:0003",
  "gene": "UniProtKB:Q9BS31",
  "gene_symbol": "ZNF649",
  "term_label": "Unknown cellular component",
  "gene_name": "Zinc finger protein 649"
}